{
  "term_id": "GO:0046933",
  "gene_name": "ATP synthase subunit epsilon, mitochondrial",
  "term_label": "proton-transporting ATP synthase activity, rotational mechanism",
  "gene_symbol": "ATP5F1E",
  "gene": "UniProtKB:P56381"
}